cysteate synthase activity [GO:0044686] (molecular function) Definition: Catalysis of the reaction: O-phospho-L-serine + sulfite + H+ = L-cysteate + phosphate. References: PMID:19761441 Sources: RHEA:26486 Relationships: is a type of transferase activity, transferring alkyl or aryl (other than methyl) groups [GO:0016765]